{
  "term_label": "sperm principal piece",
  "term_id": "GO:0097228",
  "gene_symbol": "CATSPERD",
  "gene_name": "Cation channel sperm-associated auxiliary subunit delta",
  "gene": "UniProtKB:Q86XM0"
}